{
  "term_label": "Unknown biological process",
  "gene_symbol": "ZSWIM8",
  "term_id": "UNKNOWN:0002",
  "gene_name": "Zinc finger SWIM domain-containing protein 8",
  "gene": "UniProtKB:A7E2V4"
}